regulation of response to macrophage colony-stimulating factor [GO:1903969] (biological process) Definition: Any process that modulates the frequency, rate or extent of response to macrophage colony-stimulating factor. Subtypes: GO:1903970, positive regulation of response to macrophage colony-stimulating factor [GO:1903971], regulation of cellular response to macrophage colony-stimulating factor stimulus [GO:1903972] References: PMID:19100238 Sources: GOC:BHF, GOC:TermGenie, GOC:nc, GO_REF:0000058 Also known as: regulation of response to M-CSF, regulation of response to macrophage colony-stimulating factor stimulus Relationships: is a type of regulation of response to cytokine stimulus [GO:0060759]; RO_0002211 GO:0036005